monoterpene metabolic process [GO:0043692] (biological process) Sources: Wikipedia:Monoterpene Definition: The chemical reactions and pathways involving monoterpenes, terpenes with a C10 structure. Subtypes: pinene metabolic process [GO:0033073], monoterpene biosynthetic process [GO:0043693], monoterpene catabolic process [GO:0043694] Also known as: monoterpene metabolism Relationships: is a type of terpene metabolic process [GO:0042214]